{
  "gene": "UniProtKB:Q9H2C1",
  "term_label": "regulation of transcription by RNA polymerase II",
  "gene_symbol": "LHX5",
  "gene_name": "LIM_homeobox protein Lhx5",
  "term_id": "GO:0006357"
}